{
  "gene_symbol": "CDC42SE2",
  "gene": "UniProtKB:Q9NRR3",
  "term_label": "Unknown biological process",
  "term_id": "UNKNOWN:0002",
  "gene_name": "CDC42 small effector protein 2"
}